{
  "term_label": "single-stranded RNA binding",
  "gene_symbol": "LACTB2",
  "gene": "UniProtKB:Q53H82",
  "term_id": "GO:0003727",
  "gene_name": "Endoribonuclease LACTB2"
}